positive regulation of amyloid-beta formation [GO:1902004] (biological process) Definition: Any process that activates or increases the frequency, rate or extent of amyloid-beta formation. References: PMID:17098871 Sources: GOC:TermGenie, GOC:dph Also known as: positive regulation of beta-amyloid formation, up regulation of beta-amyloid formation, up-regulation of beta-amyloid formation, upregulation of beta-amyloid formation, activation of beta-amyloid formation Relationships: is a type of GO:0034250; is a type of regulation of amyloid-beta formation [GO:1902003]; is a type of positive regulation of amyloid precursor protein catabolic process [GO:1902993]; positively regulates amyloid-beta formation [GO:0034205]